acetylcholine-induced gastric acid secretion [GO:0001699] (biological process) Definition: The regulated release of gastric acid by parietal cells in response to acetylcholine. Sources: GOC:hjd Relationships: is_a gastric acid secretion [GO:0001696]; is part of cellular response to acetylcholine [GO:1905145]; has part acetylcholine receptor activity [GO:0015464]